gel phase of basement membrane [GO:0140148] (cellular component) Relationships: is a type of external encapsulating structure [GO:0030312]; BFO_0000050 basement membrane [GO:0005604] Definition: Gel formed of proteglycans filling the basement membrane ECM space. References: PMID:21421915, PMID:28324731